{
  "term_label": "Unknown biological process",
  "gene_name": "Cilia- and flagella-associated protein 95",
  "gene_symbol": "CFAP95",
  "gene": "UniProtKB:Q5VTT2",
  "term_id": "UNKNOWN:0002"
}